{
  "gene": "UniProtKB:Q96CP6",
  "term_label": "endoplasmic reticulum-plasma membrane contact site",
  "gene_name": "Protein Aster-A",
  "gene_symbol": "GRAMD1A",
  "term_id": "GO:0140268"
}